{
  "gene": "UniProtKB:O43567",
  "gene_symbol": "RNF13",
  "term_label": "lysosomal membrane",
  "gene_name": "E3 ubiquitin-protein ligase RNF13",
  "term_id": "GO:0005765"
}